negative regulation of alpha-beta T cell proliferation [GO:0046642] (biological process) Sources: GOC:ai Relationships: is_a negative regulation of T cell proliferation [GO:0042130]; is a type of negative regulation of alpha-beta T cell activation [GO:0046636]; is a type of regulation of alpha-beta T cell proliferation [GO:0046640]; negatively regulates alpha-beta T cell proliferation [GO:0046633] Definition: Any process that stops, prevents, or reduces the frequency, rate or extent of alpha-beta T cell proliferation. Subtypes: negative regulation of NK T cell proliferation [GO:0051141], negative regulation of CD4-positive, alpha-beta T cell proliferation [GO:2000562], negative regulation of CD8-positive, alpha-beta T cell proliferation [GO:2000565] Also known as: down regulation of alpha-beta T cell proliferation, down-regulation of alpha-beta T cell proliferation, downregulation of alpha-beta T cell proliferation, negative regulation of alpha-beta T lymphocyte proliferation, negative regulation of alpha-beta T-cell proliferation, negative regulation of alpha-beta T-lymphocyte proliferation, inhibition of alpha-beta T cell proliferation